{
  "gene_symbol": "ATP5F1D",
  "term_label": "proton motive force-driven ATP synthesis",
  "term_id": "GO:0015986",
  "gene_name": "ATP synthase subunit delta, mitochondrial",
  "gene": "UniProtKB:P30049"
}